{
  "gene": "UniProtKB:Q12986",
  "gene_symbol": "NFX1",
  "term_id": "GO:0000981",
  "gene_name": "Transcriptional repressor NF-X1",
  "term_label": "DNA-binding transcription factor activity, RNA polymerase II-specific"
}